beta1-adrenergic receptor activity [GO:0004940] (molecular function) Also known as: beta1 adrenoceptor Relationships: is_a GO:0004939 Sources: GOC:mah, IUPHAR_GPCR:1274 Definition: Combining with epinephrine or norepinephrine to initiate a change in cell activity via activation of a G protein, with pharmacological characteristics of beta1-adrenergic receptors.